{
  "gene_name": "Metallothionein-1X",
  "term_id": "GO:0071276",
  "gene_symbol": "MT1X",
  "term_label": "cellular response to cadmium ion",
  "gene": "UniProtKB:P80297"
}